{
  "gene_name": "Cytoplasmic polyadenylation element-binding protein 3",
  "gene_symbol": "CPEB3",
  "term_label": "translation factor activity, RNA binding",
  "term_id": "GO:0008135",
  "gene": "UniProtKB:Q8NE35"
}